{
  "gene": "UniProtKB:Q8N4C7",
  "gene_symbol": "STX19",
  "term_label": "intracellular protein transport",
  "term_id": "GO:0006886",
  "gene_name": "Syntaxin-19"
}